{
  "gene_symbol": "ADCY9",
  "term_label": "plasma membrane",
  "gene_name": "Adenylate cyclase type 9",
  "gene": "UniProtKB:O60503",
  "term_id": "GO:0005886"
}